{
  "gene": "UniProtKB:Q8TAV0",
  "term_id": "UNKNOWN:0001",
  "gene_name": "Protein FAM76A",
  "term_label": "Unknown molecular function",
  "gene_symbol": "FAM76A"
}